thiophene-2-carbonyl-CoA monooxygenase activity [GO:0050603] (molecular function) Relationships: is a type of monooxygenase activity [GO:0004497]; is a type of oxidoreductase activity, acting on paired donors, with incorporation or reduction of molecular oxygen [GO:0016705] Definition: Catalysis of the reaction: AH(2) + O2 + thiophene-2-carbonyl-CoA = 5-hydroxythiophene-2-carbonyl-CoA + A + H2O + H+. Also known as: thiophene-2-carbonyl-CoA, hydrogen-donor:oxygen oxidoreductase activity, thiophene-2-carboxyl-CoA dehydrogenase activity, thiophene-2-carboxyl-CoA hydroxylase activity, thiophene-2-carboxyl-CoA monooxygenase activity Sources: EC:1.14.99.35, RHEA:18929